{
  "term_label": "perinuclear region of cytoplasm",
  "gene_symbol": "SYNJ2",
  "gene": "UniProtKB:O15056",
  "gene_name": "Synaptojanin-2",
  "term_id": "GO:0048471"
}